negative regulation of stress-activated protein kinase signaling cascade [GO:0070303] (BP) Relationships: is a type of GO:0070302; is a type of negative regulation of intracellular signal transduction [GO:1902532]; negatively regulates GO:0031098 Also known as: down regulation of stress-activated protein kinase signaling pathway, down-regulation of stress-activated protein kinase signaling pathway, downregulation of stress-activated protein kinase signaling pathway, negative regulation of SAPK signaling pathway, negative regulation of stress-activated protein kinase signaling pathway, negative regulation of stress-activated protein kinase signalling pathway, inhibition of stress-activated protein kinase signaling pathway Definition: Any process that stops, prevents, or reduces the frequency, rate or extent of signaling via the stress-activated protein kinase signaling cascade. Sources: GOC:mah Subtypes: negative regulation of stress-activated MAPK cascade [GO:0032873]